S-adenosyl-L-methionine:benzoic acid carboxyl methyl transferase activity [GO:0080150] (molecular function) References: PMID:10852939 Sources: MetaCyc:RXN-6722 Also known as: S-adenosyl-L-methionine:benzoate carboxyl methyltransferase activity Definition: Catalysis of the reaction: benzoate + S-adenosyl-L-methionine = methylbenzoate + S-adenosyl-L-homocysteine. Relationships: is a type of O-methyltransferase activity [GO:0008171]